{
  "gene": "UniProtKB:Q9UFW8",
  "gene_symbol": "CGGBP1",
  "gene_name": "CGG triplet repeat-binding protein 1",
  "term_label": "Unknown molecular function",
  "term_id": "UNKNOWN:0001"
}